{
  "gene_name": "4-aminobutyrate aminotransferase, mitochondrial",
  "gene_symbol": "ABAT",
  "term_id": "GO:0030170",
  "gene": "UniProtKB:P80404",
  "term_label": "pyridoxal phosphate binding"
}